filtration diaphragm [GO:0036056] (CC) References: PMID:18971929 Sources: GOC:mtg_kidney_jan10, GOC:sart Subtypes: nephrocyte diaphragm [GO:0005917], slit diaphragm [GO:0036057] Definition: A specialized cell-cell junction found between the cells of the excretory system, which provides a barrier for filtration of blood or hemolymph. Relationships: is a type of cell-cell junction [GO:0005911]